{
  "term_id": "GO:0071004",
  "gene": "UniProtKB:Q9NQ29",
  "gene_name": "Putative RNA-binding protein Luc7-like 1",
  "term_label": "U2-type prespliceosome",
  "gene_symbol": "LUC7L"
}